{
  "gene_name": "Cystatin-9",
  "gene": "UniProtKB:Q5W186",
  "term_label": "Unknown molecular function",
  "gene_symbol": "CST9",
  "term_id": "UNKNOWN:0001"
}